{
  "term_id": "GO:0005634",
  "gene_symbol": "FUBP1",
  "gene_name": "Far upstream element-binding protein 1",
  "term_label": "nucleus",
  "gene": "UniProtKB:Q96AE4"
}